ring gland development [GO:0035271] (biological process) Note: See also the fly_anatomy.ontology terms 'ring gland ; FBbt:00001722, 'prothoracic gland ; FBbt:00001724', 'corpus allatum ; FBbt:00005800' and 'corpus cardiacum ; FBbt:00005799. Definition: Progression of the ring gland over time, from its formation to a mature structure. The ring gland is a neuroendocrine organ found in higher Dipterans, which is composed of the prothoracic gland, the corpus allatum, and the corpora cardiacum. The ring gland is the site of production and release of ecdysteroids and juvenile hormones. Relationships: is a type of GO:0048732; is part of endocrine system development [GO:0035270] References: PMID:11223816, PMID:9584098 Sources: GOC:bf